negative regulation of eye photoreceptor cell development [GO:0042480] (biological process) Subtypes: negative regulation of compound eye photoreceptor development [GO:0045316] Relationships: is a type of negative regulation of cell development [GO:0010721]; is a type of regulation of eye photoreceptor cell development [GO:0042478]; negatively regulates eye photoreceptor cell development [GO:0042462] Sources: GOC:jl Definition: Any process that stops, prevents, or reduces the frequency, rate or extent of eye photoreceptor development. Also known as: down regulation of eye photoreceptor cell development, down-regulation of eye photoreceptor cell development, downregulation of eye photoreceptor cell development, negative regulation of eye photoreceptor development, inhibition of eye photoreceptor cell development